{
  "gene": "UniProtKB:Q8TAV3",
  "term_id": "GO:0005737",
  "term_label": "cytoplasm",
  "gene_symbol": "CYP2W1",
  "gene_name": "Cytochrome P450 2W1"
}